{
  "gene_name": "CREB-regulated transcription coactivator 3",
  "term_label": "cAMP response element binding protein binding",
  "gene": "UniProtKB:Q6UUV7",
  "gene_symbol": "CRTC3",
  "term_id": "GO:0008140"
}